{
  "gene_symbol": "CYB561A3",
  "gene": "UniProtKB:Q8NBI2",
  "term_id": "GO:0005765",
  "term_label": "lysosomal membrane",
  "gene_name": "Lysosomal membrane ascorbate-dependent ferrireductase CYB561A3"
}